{
  "gene": "UniProtKB:O60262",
  "gene_name": "Guanine nucleotide-binding protein G(I)_G(S)_G(O) subunit gamma-7",
  "gene_symbol": "GNG7",
  "term_label": "G-protein beta-subunit binding",
  "term_id": "GO:0031681"
}